negative regulation of response to stimulus [GO:0048585] (biological process) Relationships: is a type of negative regulation of biological process [GO:0048519]; is a type of regulation of response to stimulus [GO:0048583]; negatively regulates GO:0050896 Definition: Any process that stops, prevents, or reduces the frequency, rate or extent of a response to a stimulus. Response to stimulus is a change in state or activity of a cell or an organism (in terms of movement, secretion, enzyme production, gene expression, etc.) as a result of a stimulus. Subtypes: negative regulation of response to biotic stimulus [GO:0002832], negative regulation of signal transduction [GO:0009968], negative regulation of photomorphogenesis [GO:0010100], negative regulation of vernalization response [GO:0010221], GO:0014745, negative regulation of defense response [GO:0031348], GO:0032102, negative regulation of response to nutrient levels [GO:0032108], GO:0045738, negative regulation of establishment of competence for transformation [GO:0045808], negative regulation of short-day photoperiodism, flowering [GO:0048577], negative regulation of long-day photoperiodism, flowering [GO:0048579], negative regulation of immune response [GO:0050777], GO:0060761, negative regulation of insulin secretion involved in cellular response to glucose stimulus [GO:0061179], GO:0070571, negative regulation of response to water deprivation [GO:0080148], GO:0090288, negative regulation of thermomorphogenesis [GO:0140921], negative regulation of cellular response to heat [GO:1900035], GO:1900038, negative regulation of cellular response to alkaline pH [GO:1900068], negative regulation of cellular response to insulin stimulus [GO:1900077], GO:1900432, negative regulation of filamentous growth of a population of unicellular organisms in response to chemical stimulus [GO:1900438], negative regulation of response to pullulan [GO:1900519], negative regulation of response to amylopectin [GO:1900522], GO:1900742, GO:1901001, GO:1901181, negative regulation of response to alcohol [GO:1901420], GO:1901432, negative regulation of response to furfural [GO:1901443], negative regulation of response to benzene [GO:1901452], negative regulation of response to toluene [GO:1901455], negative regulation of response to acetate [GO:1901458], negative regulation of response to formic acid [GO:1901461], negative regulation of shade avoidance [GO:1902447], negative regulation of response to oxidative stress [GO:1902883], GO:1903035, negative regulation of fear response [GO:1903366], negative regulation of response to endoplasmic reticulum stress [GO:1903573], negative regulation of stress response to copper ion [GO:1903854], negative regulation of error-prone translesion synthesis [GO:1904332], negative regulation of telomere maintenance in response to DNA damage [GO:1904506], negative regulation of cellular response to manganese ion [GO:1905803], negative regulation of cellular response to oxidopamine [GO:1905847], GO:1905888, negative regulation of response to calcium ion [GO:1905946], GO:2000655, negative regulation of cellular response to X-ray [GO:2000684], negative regulation of detection of glucose [GO:2000971], negative regulation of response to drug [GO:2001024], GO:2001229 Also known as: down regulation of response to stimulus, down-regulation of response to stimulus, downregulation of response to stimulus, inhibition of response to stimulus Note: Note that this term is in the subset of terms that should not be used for direct gene product annotation. Instead, select a child term or, if no appropriate child term exists, please request a new term. Direct annotations to this term may be amended during annotation QC. Sources: GOC:jid